{
  "gene_symbol": "TGFB1",
  "term_label": "transforming growth factor beta receptor signaling pathway",
  "term_id": "GO:0007179",
  "gene": "UniProtKB:P01137",
  "gene_name": "Transforming growth factor beta-1 proprotein"
}